{
  "gene_name": "WW domain binding protein 1-like",
  "term_id": "GO:0038160",
  "gene": "UniProtKB:Q9NX94",
  "term_label": "CXCL12-activated CXCR4 signaling pathway",
  "gene_symbol": "WBP1L"
}